{
  "term_label": "inflammatory response",
  "gene_symbol": "IL36A",
  "gene_name": "Interleukin-36 alpha",
  "term_id": "GO:0006954",
  "gene": "UniProtKB:Q9UHA7"
}